{
  "gene": "UniProtKB:O60284",
  "gene_name": "Suppression of tumorigenicity 18 protein",
  "term_id": "GO:0005634",
  "term_label": "nucleus",
  "gene_symbol": "ST18"
}